{
  "term_label": "immune response",
  "gene_symbol": "SLAMF9",
  "term_id": "GO:0006955",
  "gene_name": "SLAM family member 9",
  "gene": "UniProtKB:Q96A28"
}